{
  "gene": "UniProtKB:Q8NFB2",
  "term_label": "Unknown cellular component",
  "term_id": "UNKNOWN:0003",
  "gene_symbol": "TMEM185A",
  "gene_name": "Transmembrane protein 185A"
}